{
  "gene_symbol": "TMEM160",
  "term_id": "UNKNOWN:0001",
  "term_label": "Unknown molecular function",
  "gene_name": "Transmembrane protein 160",
  "gene": "UniProtKB:Q9NX00"
}